{
  "term_id": "GO:0030141",
  "term_label": "secretory granule",
  "gene_symbol": "KLK3",
  "gene": "UniProtKB:P07288",
  "gene_name": "Prostate-specific antigen"
}